endoplasmic reticulum-organelle membrane tether activity [GO:0170009] (molecular function) Subtypes: mitochondrion-endoplasmic reticulum membrane tether activity [GO:0140474], GO:0140506, peroxisome-endoplasmic reticulum membrane tether activity [GO:0160229], endoplasmic reticulum-endosome tether activity [GO:0170016] References: PMID:29858488 Relationships: is a type of protein-membrane adaptor activity [GO:0043495] Definition: The binding activity of a molecule that brings together two membranes, either via membrane lipid binding or by interacting with a membrane protein, to establish or maintain membrane contact sites and mediate organelle exchange and communication.